{
  "gene_symbol": "KBTBD2",
  "gene_name": "Kelch repeat and BTB domain-containing protein 2",
  "gene": "UniProtKB:Q8IY47",
  "term_id": "GO:1990756",
  "term_label": "ubiquitin-like ligase-substrate adaptor activity"
}